{
  "gene": "UniProtKB:A0FGR9",
  "term_label": "Unknown biological process",
  "term_id": "UNKNOWN:0002",
  "gene_name": "Extended synaptotagmin-3",
  "gene_symbol": "ESYT3"
}